UDP-N-acetylmuramoylalanyl-D-glutamyl-2,6-diaminopimelate-D-alanyl-D-alanine ligase activity [GO:0008766] (molecular function) Definition: Catalysis of the reaction: ATP + UDP-N-acetylmuramoyl-L-alanyl-D-glutamyl-meso-2,6-diaminoheptanedioate + D-alanyl-D-alanine = ADP + phosphate + UDP-N-acetylmuramoyl-L-alanyl-D-glutamyl-6-carboxy-L-lysyl-D-alanyl-D-alanine. Sources: RHEA:28374 Relationships: is_a acid-amino acid ligase activity [GO:0016881]